lymphocyte anergy [GO:0002249] (BP) Sources: GOC:add Subtypes: B cell anergy [GO:0002515], T cell anergy [GO:0002870] Relationships: is a type of tolerance induction [GO:0002507] Definition: Any process contributing to lymphocyte anergy, a state of functional inactivation. Regulation: regulated by regulation of lymphocyte anergy [GO:0002911]; negatively regulated by negative regulation of lymphocyte anergy [GO:0002912]; positively regulated by positive regulation of lymphocyte anergy [GO:0002913]